{
  "term_label": "Unknown molecular function",
  "gene": "UniProtKB:Q96S96",
  "term_id": "UNKNOWN:0001",
  "gene_symbol": "PEBP4",
  "gene_name": "Phosphatidylethanolamine-binding protein 4"
}